{
  "term_id": "GO:0010629",
  "gene": "UniProtKB:O15523",
  "term_label": "negative regulation of gene expression",
  "gene_name": "ATP-dependent RNA helicase DDX3Y",
  "gene_symbol": "DDX3Y"
}